{
  "term_label": "Unknown cellular component",
  "gene": "UniProtKB:Q86UX6",
  "gene_name": "Serine_threonine-protein kinase 32C",
  "term_id": "UNKNOWN:0003",
  "gene_symbol": "STK32C"
}